cellular response to cGMP [GO:0071321] (biological process) Definition: Any process that results in a change in state or activity of a cell (in terms of movement, secretion, enzyme production, gene expression, etc.) as a result of a cGMP (cyclic GMP, guanosine 3',5'-cyclophosphate) stimulus. Relationships: is a type of response to cGMP [GO:0070305]; is a type of cellular response to nitrogen compound [GO:1901699]; is a type of cellular response to oxygen-containing compound [GO:1901701] Also known as: cellular response to 3',5' cGMP, cellular response to 3',5'-cGMP, cellular response to cyclic GMP, cellular response to guanosine 3',5'-cyclophosphate Sources: GOC:mah